{
  "term_label": "regulation of canonical Wnt signaling pathway",
  "term_id": "GO:0060828",
  "gene": "UniProtKB:Q8N7J2",
  "gene_symbol": "AMER2",
  "gene_name": "APC membrane recruitment protein 2"
}